neural tube formation [GO:0001841] (biological process) Sources: GOC:dph, ISBN:0878932437 Definition: The formation of a tube from the flat layer of ectodermal cells known as the neural plate. This will give rise to the central nervous system. Also known as: neural tube morphogenesis, neurulation Relationships: is a type of GO:0001838; is part of neural tube development [GO:0021915]